negative regulation of detection of mechanical stimulus involved in sensory perception of touch [GO:1905788] (biological process) Relationships: is a type of negative regulation of nervous system process [GO:0031645]; is a type of negative regulation of response to external stimulus [GO:0032102]; is a type of regulation of detection of mechanical stimulus involved in sensory perception of touch [GO:1905787]; negatively regulates detection of mechanical stimulus involved in sensory perception of touch [GO:0050976] Definition: Any process that stops, prevents or reduces the frequency, rate or extent of detection of mechanical stimulus involved in sensory perception of touch. Also known as: down regulation of detection of mechanical stimulus involved in sensory perception of touch, down regulation of perception of touch, detection of mechanical stimulus, down regulation of perception of touch, sensory detection of mechanical stimulus, down regulation of perception of touch, sensory transduction of mechanical stimulus, down regulation of sensory detection of mechanical stimulus during perception of touch, down regulation of sensory transduction of mechanical stimulus during perception of touch, down regulation of tactition, sensory detection of mechanical stimulus, down-regulation of detection of mechanical stimulus involved in sensory perception of touch, down-regulation of perception of touch, detection of mechanical stimulus, down-regulation of perception of touch, sensory detection of mechanical stimulus, down-regulation of perception of touch, sensory transduction of mechanical stimulus, down-regulation of sensory detection of mechanical stimulus during perception of touch, down-regulation of sensory transduction of mechanical stimulus during perception of touch, down-regulation of tactition, sensory detection of mechanical stimulus, downregulation of detection of mechanical stimulus involved in sensory perception of touch, downregulation of perception of touch, detection of mechanical stimulus, downregulation of perception of touch, sensory detection of mechanical stimulus, downregulation of perception of touch, sensory transduction of mechanical stimulus, downregulation of sensory detection of mechanical stimulus during perception of touch, downregulation of sensory transduction of mechanical stimulus during perception of touch, downregulation of tactition, sensory detection of mechanical stimulus, negative regulation of perception of touch, detection of mechanical stimulus, negative regulation of perception of touch, sensory detection of mechanical stimulus, negative regulation of perception of touch, sensory transduction of mechanical stimulus, negative regulation of sensory detection of mechanical stimulus during perception of touch, negative regulation of sensory transduction of mechanical stimulus during perception of touch, negative regulation of tactition, sensory detection of mechanical stimulus, inhibition of detection of mechanical stimulus involved in sensory perception of touch, inhibition of perception of touch, detection of mechanical stimulus, inhibition of perception of touch, sensory detection of mechanical stimulus, inhibition of perception of touch, sensory transduction of mechanical stimulus, inhibition of sensory detection of mechanical stimulus during perception of touch, inhibition of sensory transduction of mechanical stimulus during perception of touch, inhibition of tactition, sensory detection of mechanical stimulus References: PMID:8692859 Sources: GOC:TermGenie, GO_REF:0000058